{
  "gene_name": "EEF1A lysine methyltransferase 4",
  "gene": "UniProtKB:P0DPD7",
  "gene_symbol": "EEF1AKMT4",
  "term_label": "Unknown cellular component",
  "term_id": "UNKNOWN:0003"
}